{
  "term_id": "UNKNOWN:0002",
  "gene": "UniProtKB:Q7Z7F0",
  "gene_name": "KH homology domain-containing protein 4",
  "gene_symbol": "KHDC4",
  "term_label": "Unknown biological process"
}